{
  "term_label": "protein folding",
  "gene": "UniProtKB:Q5VVH2",
  "gene_symbol": "FKBP1C",
  "term_id": "GO:0006457",
  "gene_name": "Peptidyl-prolyl cis-trans isomerase FKBP1C"
}